cellular response to platinum ion [GO:0071290] (biological process) Sources: GOC:mah Definition: Any process that results in a change in state or activity of a cell (in terms of movement, secretion, enzyme production, gene expression, etc.) as a result of a platinum stimulus. Relationships: is a type of GO:0070541; is_a cellular response to metal ion [GO:0071248] Also known as: cellular response to platinum